alpha9-beta1 integrin-VEGF-D complex [GO:0071121] (cellular component) Relationships: is a type of plasma membrane protein complex [GO:0098797] Also known as: ITGA9-ITGB1-FIGF complex Definition: A protein complex that consists of an alpha9-beta1 integrin complex bound to vascular endothelial growth factor D. References: PMID:15590642